alpha-(1,2)-fucosyltransferase activity [GO:0031127] (MF) Relationships: is a type of fucosyltransferase activity [GO:0008417] Subtypes: GO:0008107 Also known as: alpha-(1->2)-fucosyltransferase activity, alpha-1,2-fucosyltransferase activity Definition: Catalysis of the transfer of an L-fucosyl group from GDP-beta-L-fucose to an acceptor molecule to form an alpha-(1->2) linkage. Sources: GOC:mah